{
  "gene": "UniProtKB:Q8TE23",
  "term_label": "sweet taste receptor complex",
  "term_id": "GO:1903767",
  "gene_name": "Taste receptor type 1 member 2",
  "gene_symbol": "TAS1R2"
}